{
  "gene": "UniProtKB:Q16602",
  "gene_symbol": "CALCRL",
  "term_label": "adrenomedullin receptor activity",
  "gene_name": "Calcitonin gene-related peptide type 1 receptor",
  "term_id": "GO:0001605"
}